histone H3K18 ubiquitin ligase activity [GO:0140248] (molecular function) Definition: Catalysis of the transfer of a ubiquitin molecule to histone 3 at the lysine-18 residue. References: PMID:27595565 Note: Comment: Note that the residue position corresponds to the canonical human H3 histone (UniProtKB:P84243); this residue is conserved across all eukaryotes. Residue 1 is the first residue following removal of the initiating Methionine (Met). Note that each histone is encoded by multiple genes, and sequences may vary across different genes within an organism. Relationships: is a type of histone H3 ubiquitin ligase activity [GO:0141055]